{
  "term_label": "Unknown molecular function",
  "gene_name": "Proteoglycan 4",
  "gene_symbol": "PRG4",
  "gene": "UniProtKB:Q92954",
  "term_id": "UNKNOWN:0001"
}